oviduct development [GO:0060066] (biological process) Definition: The reproductive developmental process whose specific outcome is the progression of an oviduct over time, from its formation to the mature structure. An oviduct is a tube through which an ova passes from the ovary to the uterus, or from the ovary to the outside of the organism. References: PMID:22918811, PMID:27875265 Sources: GOC:dph, GOC:ebc Also known as: fallopian tube development, Mullerian tract development Relationships: is a type of tube development [GO:0035295]; is_a reproductive structure development [GO:0048608]